{
  "term_label": "ribosomal small subunit export from nucleus",
  "gene": "UniProtKB:O14980",
  "gene_symbol": "XPO1",
  "gene_name": "Exportin-1",
  "term_id": "GO:0000056"
}